{
  "gene_symbol": "HLA-DMB",
  "gene_name": "HLA class II histocompatibility antigen, DM beta chain",
  "gene": "UniProtKB:P28068",
  "term_id": "GO:0050778",
  "term_label": "positive regulation of immune response"
}